regulation of primary heart field cardioblast proliferation [GO:0003265] (biological process) Definition: Any process that modulates the frequency, rate or extent of cardioblast proliferation in the primary heart field. A cardioblast is a cardiac precursor cell. It is a cell that has been committed to a cardiac fate, but will undergo more cell division rather than terminally differentiating. In mammals the primary heart field gives rise to the left ventricle. Sources: GOC:mtg_heart, GOC:rl Relationships: is a type of regulation of cardioblast proliferation [GO:0003264] Also known as: regulation of FHF cardioblast proliferation, regulation of first heart field cardioblast proliferation, regulation of first heart field cardiac proliferation